{
  "gene_name": "Inactive C-alpha-formylglycine-generating enzyme 2",
  "term_label": "endoplasmic reticulum",
  "gene": "UniProtKB:Q8NBJ7",
  "term_id": "GO:0005783",
  "gene_symbol": "SUMF2"
}